(+)-trans-carveol dehydrogenase activity [GO:0033702] (MF) Also known as: (+)-trans-carveol:NAD+ oxidoreductase activity Sources: EC:1.1.1.275, RHEA:14825 Relationships: is a type of oxidoreductase activity, acting on the CH-OH group of donors, NAD or NADP as acceptor [GO:0016616] Definition: Catalysis of the reaction: (1R,5S)-carveol + NAD+ = (S)-carvone + H+ + NADH.